{
  "term_label": "Unknown biological process",
  "gene_symbol": "TRAJ54",
  "term_id": "UNKNOWN:0002",
  "gene_name": "T cell receptor alpha joining 54 (Fragment)",
  "gene": "UniProtKB:A0A075B712"
}